{
  "term_label": "regulation of gene expression",
  "gene_name": "Nuclear nucleic acid-binding protein C1D",
  "gene": "UniProtKB:Q13901",
  "gene_symbol": "C1D",
  "term_id": "GO:0010468"
}